{
  "term_id": "GO:0005737",
  "gene_name": "Glutathione S-transferase theta-2",
  "term_label": "cytoplasm",
  "gene": "UniProtKB:P0CG29",
  "gene_symbol": "GSTT2"
}